hydroquinone binding [GO:1902314] (MF) Also known as: quinol binding Relationships: is a type of GO:0005488 References: PMID:15667223 Sources: GOC:TermGenie, GOC:bhm Definition: Binding to hydroquinone.